{
  "term_label": "adherens junction",
  "gene": "UniProtKB:Q13796",
  "term_id": "GO:0005912",
  "gene_symbol": "SHROOM2",
  "gene_name": "Protein Shroom2"
}